{
  "term_id": "GO:0015252",
  "term_label": "proton channel activity",
  "gene_name": "Proton channel OTOP3",
  "gene_symbol": "OTOP3",
  "gene": "UniProtKB:Q7RTS5"
}